{
  "gene_symbol": "CDCA8",
  "gene_name": "Borealin",
  "term_id": "GO:0000775",
  "gene": "UniProtKB:Q53HL2",
  "term_label": "chromosome, centromeric region"
}